{
  "term_label": "nucleotide-excision repair",
  "gene_name": "General transcription factor IIH subunit 2-like protein",
  "gene": "UniProtKB:Q6P1K8",
  "term_id": "GO:0006289",
  "gene_symbol": "GTF2H2C"
}